12-oxophytodienoate reductase activity [GO:0016629] (molecular function) Relationships: is a type of oxidoreductase activity, acting on the CH-CH group of donors, NAD or NADP as acceptor [GO:0016628] Sources: EC:1.3.1.42, RHEA:21888 Definition: Catalysis of the reaction: 8-[(1R,2R)-3-oxo-2-{(Z)-pent-2-en-1-yl}cyclopentyl]octanoate + NADP+ = (15Z)-12-oxophyto-10,15-dienoate + H+ + NADPH. Also known as: 12-oxo-phytodienoate reductase activity, 12-oxo-phytodienoic acid reductase activity, 8-[(1R,2R)-3-oxo-2-{(Z)-pent-2-enyl}cyclopentyl]octanoate:NADP+ 4-oxidoreductase activity